{
  "gene_name": "WAP, Kazal, immunoglobulin, Kunitz and NTR domain-containing protein 1",
  "gene": "UniProtKB:Q96NZ8",
  "term_id": "GO:0005615",
  "gene_symbol": "WFIKKN1",
  "term_label": "extracellular space"
}